{
  "term_label": "Unknown molecular function",
  "term_id": "UNKNOWN:0001",
  "gene_symbol": "HERVK_113",
  "gene": "UniProtKB:Q902F9",
  "gene_name": "Endogenous retrovirus group K member 113 Env polyprotein"
}